{
  "gene": "UniProtKB:Q5XKL5",
  "term_id": "UNKNOWN:0001",
  "term_label": "Unknown molecular function",
  "gene_symbol": "BTBD8",
  "gene_name": "BTB_POZ domain-containing protein 8"
}